{
  "gene_symbol": "SMIM38",
  "term_id": "UNKNOWN:0002",
  "gene_name": "Small integral membrane protein 38",
  "term_label": "Unknown biological process",
  "gene": "UniProtKB:A0A286YFK9"
}